{
  "gene": "UniProtKB:Q96NB3",
  "gene_name": "Zinc finger protein 830",
  "gene_symbol": "ZNF830",
  "term_id": "GO:0033260",
  "term_label": "nuclear DNA replication"
}